{
  "gene_name": "Pleckstrin homology domain-containing family G member 4B",
  "gene": "UniProtKB:Q96PX9",
  "gene_symbol": "PLEKHG4B",
  "term_id": "GO:0005737",
  "term_label": "cytoplasm"
}